axoneme assembly [GO:0035082] (biological process) Note: Note that cilia and eukaryotic flagella are deemed to be equivalent. Sources: GOC:bf, GOC:cilia, GOC:jl, ISBN:0815316194 Also known as: ciliary axoneme assembly, cilium axoneme assembly, flagellar axoneme assembly, flagellum axoneme assembly, axoneme biogenesis, cilium axoneme biogenesis Subtypes: GO:0007288 Definition: The assembly and organization of an axoneme, the bundle of microtubules and associated proteins that forms the core of cilia (also called flagella) in eukaryotic cells and is responsible for their movements. Relationships: is_a microtubule bundle formation [GO:0001578]; is_a cellular component assembly [GO:0022607]; is part of cilium assembly [GO:0060271]